{
  "term_label": "calcium ion binding",
  "term_id": "GO:0005509",
  "gene_name": "Protein S100-A11",
  "gene": "UniProtKB:P31949",
  "gene_symbol": "S100A11"
}